P-type potassium transmembrane transporter activity [GO:0008556] (molecular function) Sources: RHEA:16777 Subtypes: P-type sodium:potassium-exchanging transporter activity [GO:0005391], P-type potassium:proton transporter activity [GO:0008900] Definition: Enables the transfer of a solute or solutes from one side of a membrane to the other according to the reaction: ATP + H2O + K+(out) = ADP + phosphate + K+(in). Also known as: ATP-dependent potassium transmembrane transporter activity, K+-transporting ATPase activity, potassium transmembrane transporter activity, phosphorylative mechanism, potassium transporting ATPase activity, potassium-transporting ATPase activity, potassium-uptake-ATPase activity, K(+)-importing ATPase activity, potassium ABC transporter, potassium-importing ATPase activity, ATP phosphohydrolase (K+-importing), ATPase-coupled potassium transmembrane transporter activity, K(+)-transporting ATPase activity, K+-importing ATPase activity Relationships: is_a potassium ion transmembrane transporter activity [GO:0015079]; is a type of P-type ion transporter activity [GO:0015662]; is a type of ATPase-coupled monoatomic cation transmembrane transporter activity [GO:0019829]